{
  "gene_symbol": "SERINC2",
  "term_label": "Unknown biological process",
  "term_id": "UNKNOWN:0002",
  "gene": "UniProtKB:Q96SA4",
  "gene_name": "Serine incorporator 2"
}